{
  "gene_name": "Translin",
  "gene_symbol": "TSN",
  "term_label": "cytoplasm",
  "gene": "UniProtKB:Q15631",
  "term_id": "GO:0005737"
}